{
  "gene_symbol": "SHC1",
  "term_id": "GO:0030971",
  "gene": "UniProtKB:P29353",
  "gene_name": "SHC-transforming protein 1",
  "term_label": "receptor tyrosine kinase binding"
}